{
  "gene_symbol": "LCA10",
  "gene_name": "Putative lung carcinoma-associated protein 10",
  "term_id": "UNKNOWN:0003",
  "gene": "UniProtKB:Q71F78",
  "term_label": "Unknown cellular component"
}